5'-adenylyl sulfate transmembrane transporter activity [GO:1902557] (molecular function) Relationships: is_a adenine nucleotide transmembrane transporter activity [GO:0000295]; is_a GO:0005346; is_a GO:1901682; is part of GO:1902558 Note: An example of this is the YPR011C gene product in S. cerevisiae in PMID:24296033. Definition: Enables the transfer of 5'-adenylyl sulfate from one side of a membrane to the other. References: PMID:24296033 Sources: GOC:TermGenie